regulation of mRNA stability involved in response to stress [GO:0010610] (biological process) Sources: GOC:dph, GOC:tb Subtypes: regulation of mRNA stability involved in response to oxidative stress [GO:2000815] Relationships: is a type of regulation of mRNA stability [GO:0043488]; is part of cellular response to stress [GO:0033554] Definition: Any process that modulates the propensity of mRNA molecules to degradation that is part of a change in state or activity of a cell as a result of an exogenous disturbance.